{
  "gene_name": "Probable ATP-dependent RNA helicase DDX43",
  "gene_symbol": "DDX43",
  "term_id": "UNKNOWN:0002",
  "gene": "UniProtKB:Q9NXZ2",
  "term_label": "Unknown biological process"
}